{
  "gene": "UniProtKB:O75496",
  "gene_symbol": "GMNN",
  "term_id": "GO:0030174",
  "gene_name": "Geminin",
  "term_label": "regulation of DNA-templated DNA replication initiation"
}